{
  "term_id": "GO:0004930",
  "gene_symbol": "P2RY10",
  "gene_name": "Putative P2Y purinoceptor 10",
  "term_label": "G protein-coupled receptor activity",
  "gene": "UniProtKB:O00398"
}